{
  "term_id": "GO:0005634",
  "gene_name": "Tigger transposable element-derived protein 4",
  "gene_symbol": "TIGD4",
  "gene": "UniProtKB:Q8IY51",
  "term_label": "nucleus"
}